{
  "gene": "UniProtKB:P18858",
  "gene_name": "DNA ligase 1",
  "term_label": "nucleus",
  "term_id": "GO:0005634",
  "gene_symbol": "LIG1"
}